{
  "gene_name": "Thyrotropin-releasing hormone-degrading ectoenzyme",
  "gene": "UniProtKB:Q9UKU6",
  "term_label": "extracellular space",
  "gene_symbol": "TRHDE",
  "term_id": "GO:0005615"
}